mannosyl-oligosaccharide 1,3-alpha-mannosidase activity [GO:0052768] (molecular function) References: PMID:1849817, PMID:2338081 Sources: GOC:mengo_curators Relationships: is a type of mannosyl-oligosaccharide mannosidase activity [GO:0015924] Also known as: 1,3-alpha-mannosidase activity, alpha-1,3-mannosidase activity, 1,3-alpha-mannosyl-oligosaccharide alpha-D-mannohydrolase activity, alpha-1,3-mannosyl-oligosaccharide alpha-D-mannohydrolase activity Definition: Catalysis of the hydrolysis of the alpha-(1->3) bonds of alpha-D-mannose residues in mannosyl-oligosaccharide.